ascospore-type prospore assembly [GO:0031321] (biological process) Relationships: is a type of developmental process involved in reproduction [GO:0003006]; is a type of GO:0010927; is a type of GO:1903046; is part of ascospore formation [GO:0030437] References: PMID:14702385 Sources: GOC:mah Also known as: ascospore-type prospore formation, forespore formation Definition: During ascospore formation, the process in which each haploid nucleus becomes encapsulated by a double membrane.